negative regulation of lipoprotein lipase activity [GO:0051005] (biological process) Definition: Any process that stops or reduces the activity of the enzyme lipoprotein lipase. Relationships: is a type of GO:0060192; negatively regulates lipoprotein lipase activity [GO:0004465] Sources: GOC:ai Also known as: down regulation of lipoprotein lipase activity, down-regulation of lipoprotein lipase activity, downregulation of lipoprotein lipase activity, inhibition of lipoprotein lipase activity